hydroxymethylglutaryl-CoA synthase activity [GO:0004421] (MF) Definition: Catalysis of the reaction: acetoacetyl-CoA + acetyl-CoA + H2O = (S)-3-hydroxy-3-methylglutaryl-CoA + CoA + H+. Sources: RHEA:10188 Also known as: (S)-3-hydroxy-3-methylglutaryl-CoA acetoacetyl-CoA-lyase (CoA-acetylating), (s)-3-hydroxy-3-methylglutaryl-CoA acetoacetyl-CoA-lyase (CoA- acetylating) activity, 3-hydroxy-3-methylglutaryl CoA synthetase activity, 3-hydroxy-3-methylglutaryl coenzyme A synthase activity, 3-hydroxy-3-methylglutaryl coenzyme A synthetase activity, 3-hydroxy-3-methylglutaryl-CoA synthase activity, 3-hydroxy-3-methylglutaryl-coenzyme A synthase activity, HMG-CoA synthase activity, acetoacetyl coenzyme A transacetase activity, acetyl-CoA:acetoacetyl-CoA C-acetyltransferase (thioester-hydrolysing, carboxymethyl-forming), beta-hydroxy-beta-methylglutaryl-CoA synthase activity, hydroxymethylglutaryl coenzyme A synthase activity, hydroxymethylglutaryl coenzyme A-condensing enzyme, hydroxymethylglutaryl coenzyme alpha-condensing enzyme activity Relationships: is a type of acyltransferase activity, acyl groups converted into alkyl on transfer [GO:0046912]